{
  "term_id": "GO:0022857",
  "term_label": "transmembrane transporter activity",
  "gene": "UniProtKB:Q9BY10",
  "gene_name": "Thymic stromal cotransporter homolog",
  "gene_symbol": "SLC46A2"
}